{
  "term_label": "sodium-dependent phosphate transport",
  "gene_symbol": "SLC34A2",
  "gene_name": "Sodium-dependent phosphate transport protein 2B",
  "term_id": "GO:0044341",
  "gene": "UniProtKB:O95436"
}